{
  "gene_name": "Interferon alpha-17",
  "gene_symbol": "IFNA17",
  "gene": "UniProtKB:P01571",
  "term_label": "humoral immune response",
  "term_id": "GO:0006959"
}